{
  "gene_name": "ICOS ligand",
  "term_id": "GO:0050852",
  "term_label": "T cell receptor signaling pathway",
  "gene": "UniProtKB:O75144",
  "gene_symbol": "ICOSLG"
}